macromolecule biosynthetic process [GO:0009059] (biological process) Sources: GOC:mah Regulation: RO_0002211 by GO:0010556; positively regulated by GO:0010557; negatively regulated by negative regulation of macromolecule biosynthetic process [GO:0010558] Also known as: biopolymer biosynthetic process, macromolecule anabolism, macromolecule biosynthesis, macromolecule formation, macromolecule synthesis Note: Note that this term is in the subset of terms that should not be used for direct gene product annotation. Instead, select a child term or, if no appropriate child term exists, please request a new term. Direct annotations to this term may be amended during annotation QC. Subtypes: polysaccharide biosynthetic process [GO:0000271], aminoglycan biosynthetic process [GO:0006023], GO:0006412, translational elongation [GO:0006414], glycoprotein biosynthetic process [GO:0009101], colanic acid biosynthetic process [GO:0009242], amylopectin biosynthetic process [GO:0010021], cutin biosynthetic process [GO:0010143], gene expression [GO:0010467], rhodopsin biosynthetic process [GO:0016063], holo-[acyl-carrier-protein] biosynthetic process [GO:0031108], GO:0036489, lipoprotein biosynthetic process [GO:0042158], hemoglobin biosynthetic process [GO:0042541], biotin carboxyl carrier protein biosynthetic process [GO:0042966], amyloid precursor protein biosynthetic process [GO:0042983], cell wall macromolecule biosynthetic process [GO:0044038], integrin biosynthetic process [GO:0045112], GO:0045341, MHC class II biosynthetic process [GO:0045342], poly-gamma-glutamate biosynthetic process [GO:0070501], membrane macromolecule biosynthetic process [GO:0071710], GO:0141187, GO:0160307, cytochrome biosynthetic process [GO:1903605], GO:1990145 Definition: The chemical reactions and pathways resulting in the formation of a macromolecule, any molecule of high relative molecular mass, the structure of which essentially comprises the multiple repetition of units derived, actually or conceptually, from molecules of low relative molecular mass. Relationships: is a type of biosynthetic process [GO:0009058]; is a type of macromolecule metabolic process [GO:0043170]